cis-regulatory region sequence-specific DNA binding [GO:0000987] (molecular function) Subtypes: RNA polymerase II cis-regulatory region sequence-specific DNA binding [GO:0000978], GO:0000992 Sources: GOC:txnOH-2018 Also known as: bacterial-type RNA polymerase core promoter proximal region sequence-specific DNA binding, bacterial-type RNA polymerase enhancer sequence-specific DNA binding, bacterial-type RNA polymerase upstream activating sequence (UAS) sequence-specific DNA binding, bacterial-type cis-regulatory region sequence-specific DNA binding, bacterial-type proximal promoter sequence-specific DNA binding, core promoter proximal region DNA binding, core promoter proximal region sequence-specific DNA binding, eubacterial-type RNA polymerase regulatory transcription factor sequence-specific DNA binding, promoter proximal region sequence-specific DNA binding, proximal promoter sequence-specific DNA binding, cis-regulatory region binding, enhancer binding, enhancer sequence-specific DNA binding Definition: Binding to a specific upstream regulatory DNA sequence (transcription factor recognition sequence or binding site, located in cis relative to the transcription start site (i.e., on the same strand of DNA) of a gene transcribed by some RNA polymerase. Cis-regulatory sites are often referred to as a sequence motifs, enhancers, or silencers. Relationships: is a type of transcription cis-regulatory region binding [GO:0000976]